{
  "term_id": "GO:0006488",
  "gene_symbol": "ALG2",
  "gene_name": "Alpha-1,3_1,6-mannosyltransferase ALG2",
  "gene": "UniProtKB:Q9H553",
  "term_label": "dolichol-linked oligosaccharide biosynthetic process"
}